inositol-1,4-bisphosphate 1-phosphatase activity [GO:0004441] (molecular function) Definition: Catalysis of the reaction: 1D-myo-inositol 1,4-bisphosphate + H2O = 1D-myo-inositol 4-phosphate + phosphate. Also known as: inositol polyphosphate 1-phosphatase activity, 1D-myo-inositol-1,4-bisphosphate 1-phosphohydrolase activity, inositol-polyphosphate 1-phosphatase activity Sources: EC:3.1.3.57, GOC:hb Relationships: is_a inositol bisphosphate phosphatase activity [GO:0016312]